U2-type post-mRNA release spliceosomal complex [GO:0071008] (cellular component) References: PMID:19239890 Sources: GOC:ab, GOC:krc, GOC:mah, ISBN:0879695897, ISBN:0879697393 Also known as: U2/U5/U6 snRNP complex, U2/U5/U6 tri-snRNP complex, major post-mRNA release spliceosomal complex, GT-AG post-mRNA release spliceosomal complex, mammalian U2-type spliceosomal complex I Relationships: is a type of GO:0005684; is a type of post-mRNA release spliceosomal complex [GO:0071014]; BFO_0000051 U6 snRNP [GO:0005688] Definition: A spliceosomal complex that is formed following the release of the spliced product from the post-spliceosomal complex and contains the excised intron and the U2, U5 and U6 snRNPs.